{
  "term_id": "GO:0051015",
  "gene_symbol": "MYO16",
  "gene_name": "Unconventional myosin-XVI",
  "term_label": "actin filament binding",
  "gene": "UniProtKB:Q9Y6X6"
}